{
  "gene_name": "Enoyl-CoA hydratase domain-containing protein 3, mitochondrial",
  "term_label": "hydro-lyase activity",
  "gene_symbol": "ECHDC3",
  "gene": "UniProtKB:Q96DC8",
  "term_id": "GO:0016836"
}